{
  "term_id": "GO:0097526",
  "gene_symbol": "SNRPD1",
  "gene_name": "Small nuclear ribonucleoprotein Sm D1",
  "term_label": "spliceosomal tri-snRNP complex",
  "gene": "UniProtKB:P62314"
}